aflatoxin catabolic process [GO:0046223] (biological process) Relationships: is a type of mycotoxin catabolic process [GO:0043387]; is a type of aflatoxin metabolic process [GO:0046222] Also known as: aflatoxin breakdown, aflatoxin catabolism, aflatoxin degradation References: PMID:20807200 Sources: GOC:ai Definition: The chemical reactions and pathways resulting in the breakdown of aflatoxin, a fungal metabolite found as a contaminant in moldy grains that induces liver cancer. Aflatoxin induces a G to T transversion at codon 249 of p53, leading to its inactivation. Aflatoxin is converted to a chemical carcinogen by P450.